{
  "gene_name": "Kinetochore protein Spc24",
  "term_id": "GO:0008017",
  "term_label": "microtubule binding",
  "gene": "UniProtKB:Q8NBT2",
  "gene_symbol": "SPC24"
}